{
  "gene_name": "Arrestin domain-containing protein 5",
  "term_label": "plasma membrane",
  "term_id": "GO:0005886",
  "gene_symbol": "ARRDC5",
  "gene": "UniProtKB:A6NEK1"
}